{
  "gene_symbol": "Q8NBF4",
  "gene": "UniProtKB:Q8NBF4",
  "gene_name": "Putative uncharacterized protein FLJ33307",
  "term_label": "Unknown cellular component",
  "term_id": "UNKNOWN:0003"
}